{
  "gene": "UniProtKB:Q8TCT7",
  "term_id": "GO:0005765",
  "gene_name": "Signal peptide peptidase-like 2B",
  "gene_symbol": "SPPL2B",
  "term_label": "lysosomal membrane"
}